{
  "term_id": "GO:0003917",
  "gene_name": "DNA topoisomerase 1",
  "gene": "UniProtKB:P11387",
  "term_label": "DNA topoisomerase type I (single strand cut, ATP-independent) activity",
  "gene_symbol": "TOP1"
}